{
  "gene_name": "Tropomyosin beta chain",
  "term_id": "GO:0051015",
  "gene_symbol": "TPM2",
  "gene": "UniProtKB:P07951",
  "term_label": "actin filament binding"
}